{
  "gene_name": "Heparan-sulfate 6-O-sulfotransferase 1",
  "gene_symbol": "HS6ST1",
  "term_id": "GO:0017095",
  "gene": "UniProtKB:O60243",
  "term_label": "heparan sulfate 6-sulfotransferase activity"
}